flocculation [GO:0000128] (biological process) Note: The word floc derives from the Latin word floccus, which means a tuft of wool. Relationships: is a type of biological process involved in intraspecies interaction between organisms [GO:0051703]; is a type of adhesion between unicellular organisms [GO:0098610] Subtypes: galactose-specific flocculation [GO:0036349], mannose-specific flocculation [GO:0036350] References: PMID:11472912, PMID:21114594, PMID:8740415 Sources: GOC:jl, GOC:vw Also known as: cell-cell adhesion involved in flocculation, cell-cell adhesion involved in flocculation via cell wall protein-carbohydrate interaction, co-flocculation, coflocculation, coflocculation via lectin-mannose interaction, coflocculation via protein-carbohydrate interaction, flocculation via cell wall protein-carbohydrate interaction, flocculation via extracellular polymer Regulation: regulated by GO:0060256; negatively regulated by negative regulation of flocculation [GO:0060257]; RO_0002213 by GO:1900735 Definition: The reversible, non-sexual aggregation of single-celled organisms in suspension to form aggregates of many cells known as flocs.